sorbitol metabolic process [GO:0006060] (BP) Subtypes: sorbitol biosynthetic process [GO:0006061], sorbitol catabolic process [GO:0006062] Sources: ISBN:0198506732 Relationships: is a type of hexitol metabolic process [GO:0006059] Definition: The chemical reactions and pathways involving sorbitol (D-glucitol), one of the ten stereoisomeric hexitols. It can be derived from glucose by reduction of the aldehyde group. Also known as: sorbitol metabolism